{
  "gene": "UniProtKB:Q8WXX5",
  "term_label": "cytoplasm",
  "gene_symbol": "DNAJC9",
  "term_id": "GO:0005737",
  "gene_name": "DnaJ homolog subfamily C member 9"
}